{
  "gene_symbol": "MAPKAPK2",
  "term_label": "calcium-dependent protein serine/threonine kinase activity",
  "term_id": "GO:0009931",
  "gene_name": "MAP kinase-activated protein kinase 2",
  "gene": "UniProtKB:P49137"
}